protein-bilin linkage [GO:0017007] (biological process) Sources: GOC:ai Subtypes: protein-phycobiliviolin linkage [GO:0017008], protein-phycocyanobilin linkage [GO:0017009], protein-phycourobilin linkage [GO:0017010], protein-phycoerythrobilin linkage [GO:0017011], protein-phytochromobilin linkage [GO:0017012] Relationships: is a type of protein-tetrapyrrole linkage [GO:0017006] Definition: The covalent linkage of bilin and a protein.